adenosine 3',5'-bisphosphate transmembrane transport [GO:0071106] (biological process) Note: Note that this term is not intended for use in annotating lateral movement within membranes. Definition: The process in which adenosine 3',5'-bisphosphate is transported across a membrane. Sources: GOC:mah Also known as: adenosine 3',5'-bisphosphate membrane transport, adenosine 3',5'-diphosphate transport, adenosine 3'-phosphate-5'-phosphate transmembrane transport Relationships: is a type of purine ribonucleotide transport [GO:0015868]; is a type of adenine nucleotide transport [GO:0051503]; is a type of GO:0072530; is_a nucleotide transmembrane transport [GO:1901679]